{
  "term_label": "magnesium ion homeostasis",
  "gene_symbol": "CNNM2",
  "term_id": "GO:0010960",
  "gene": "UniProtKB:Q9H8M5",
  "gene_name": "Metal transporter CNNM2"
}